{
  "gene_name": "Angiogenin",
  "term_id": "GO:0050830",
  "gene_symbol": "ANG",
  "term_label": "defense response to Gram-positive bacterium",
  "gene": "UniProtKB:P03950"
}